{
  "gene_name": "Protein MAK16 homolog",
  "gene": "UniProtKB:Q9BXY0",
  "term_label": "maturation of 5.8S rRNA",
  "term_id": "GO:0000460",
  "gene_symbol": "MAK16"
}